{
  "term_id": "GO:0071280",
  "gene_symbol": "PRNP",
  "gene_name": "Major prion protein",
  "term_label": "cellular response to copper ion",
  "gene": "UniProtKB:P04156"
}